negative regulation of retinoic acid receptor signaling pathway [GO:0048387] (biological process) Sources: GOC:dgh Also known as: down regulation of retinoic acid receptor signaling pathway, down-regulation of retinoic acid receptor signaling pathway, downregulation of retinoic acid receptor signaling pathway, negative regulation of RAR signaling pathway, negative regulation of RAR signalling pathway, negative regulation of retinoic acid receptor signalling pathway, inhibition of retinoic acid receptor signaling pathway Relationships: is a type of regulation of retinoic acid receptor signaling pathway [GO:0048385]; is a type of negative regulation of intracellular signal transduction [GO:1902532]; negatively regulates GO:0048384 Definition: Any process that stops, prevents, or reduces the frequency, rate or extent of retinoic acid receptor signaling pathway activity.